{
  "gene_name": "Transcription factor JunD",
  "term_id": "GO:0048545",
  "term_label": "response to steroid hormone",
  "gene_symbol": "JUND",
  "gene": "UniProtKB:P17535"
}